{
  "gene_name": "Probable E3 ubiquitin-protein ligase HECTD4",
  "gene": "UniProtKB:Q9Y4D8",
  "gene_symbol": "HECTD4",
  "term_id": "UNKNOWN:0001",
  "term_label": "Unknown molecular function"
}